{
  "term_label": "serotonin-gated cation-selective signaling pathway",
  "term_id": "GO:0140227",
  "gene_symbol": "HTR3C",
  "gene_name": "5-hydroxytryptamine receptor 3C",
  "gene": "UniProtKB:Q8WXA8"
}